{
  "term_label": "endoplasmic reticulum lumen",
  "gene_name": "Torsin-4A",
  "gene_symbol": "TOR4A",
  "gene": "UniProtKB:Q9NXH8",
  "term_id": "GO:0005788"
}